nitric oxide binding [GO:0070026] (molecular function) Definition: Binding to nitric oxide (NO). Relationships: is_a GO:0036094 Also known as: NO binding, nitrogen monoxide binding, nitrosyl binding Sources: GOC:ecd